{
  "gene_name": "Apolipoprotein C-III",
  "gene_symbol": "APOC3",
  "term_id": "GO:0010916",
  "gene": "UniProtKB:P02656",
  "term_label": "negative regulation of very-low-density lipoprotein particle clearance"
}